{
  "gene_name": "Prenylcysteine oxidase-like",
  "gene": "UniProtKB:Q8NBM8",
  "gene_symbol": "PCYOX1L",
  "term_id": "GO:0001735",
  "term_label": "prenylcysteine oxidase activity"
}